peptidoglycan-based cell wall organization [GO:0031504] (biological process) Also known as: peptidoglycan-based cell wall organisation, peptidoglycan-based cell wall organization and biogenesis Definition: A process that is carried out at the cellular level which results in the assembly, arrangement of constituent parts, or disassembly of the peptidoglycan-based cell wall. Relationships: is a type of cell wall organization [GO:0071555] Sources: GOC:dph, GOC:jl, GOC:mah, GOC:mtg_sensu